regulation of spindle organization [GO:0090224] (biological process) Relationships: is a type of GO:0010564; is a type of regulation of microtubule cytoskeleton organization [GO:0070507]; regulates spindle organization [GO:0007051] Sources: GOC:ascb_2009, GOC:dph, GOC:tb Subtypes: negative regulation of astral microtubule depolymerization [GO:0032932], regulation of mitotic spindle organization [GO:0060236], GO:0090169 Definition: Any process that modulates the rate, frequency or extent of the assembly, arrangement of constituent parts, or disassembly of the microtubule spindle. Also known as: regulation of spindle organisation